{
  "term_label": "cytoskeleton",
  "gene_symbol": "ADD1",
  "gene": "UniProtKB:P35611",
  "term_id": "GO:0005856",
  "gene_name": "Alpha-adducin"
}